positive regulation of nicotine catabolic process [GO:0160160] (biological process) Definition: Any process that activates or increases the frequency, rate or extent of nicotine catabolic process. Relationships: is a type of positive regulation of catabolic process [GO:0009896]; positively regulates nicotine catabolic process [GO:0019608] References: PMID:15838033